positive regulation of leaflet formation by auxin mediated signaling pathway [GO:0090015] (biological process) Definition: Any process that increases the frequency, rate or extent of leaflet formation as a result of the series of molecular signals generated in response to detection of auxin. Sources: GOC:dph, GOC:sdb_2009, GOC:tb Also known as: positive regulation of leaflet formation by auxin mediated signalling pathway Relationships: is a type of GO:0009734; is a type of GO:0090016; is a type of positive regulation of leaf development [GO:1905623]; positively regulates leaflet formation [GO:0090014]